retrograde protein transport, ER to cytosol [GO:0030970] (biological process) Definition: The directed movement of unfolded or misfolded proteins from the endoplasmic reticulum to the cytosol through the translocon. References: PMID:11994744 Also known as: protein dislocation from ER, protein retrotranslocation, ER to cytosol, retrograde protein transport, endoplasmic reticulum to cytosol Relationships: is a type of protein exit from endoplasmic reticulum [GO:0032527]; is a type of endoplasmic reticulum to cytosol transport [GO:1903513]; is part of ERAD pathway [GO:0036503] Regulation: regulated by regulation of retrograde protein transport, ER to cytosol [GO:1904152]; RO_0002212 by negative regulation of retrograde protein transport, ER to cytosol [GO:1904153]; positively regulated by positive regulation of retrograde protein transport, ER to cytosol [GO:1904154]